{
  "term_id": "GO:0005794",
  "gene_symbol": "WDR77",
  "gene": "UniProtKB:Q9BQA1",
  "term_label": "Golgi apparatus",
  "gene_name": "Methylosome protein WDR77"
}